{
  "gene_name": "Zinc finger protein interacting with ribonucleoprotein K",
  "term_id": "GO:0005634",
  "term_label": "nucleus",
  "gene_symbol": "ZIK1",
  "gene": "UniProtKB:Q3SY52"
}